{
  "gene": "UniProtKB:Q9Y5X1",
  "term_label": "endocytosis",
  "gene_name": "Sorting nexin-9",
  "term_id": "GO:0006897",
  "gene_symbol": "SNX9"
}